{
  "gene": "UniProtKB:Q96LT9",
  "gene_name": "RNA-binding region-containing protein 3",
  "term_id": "GO:0005689",
  "term_label": "U12-type spliceosomal complex",
  "gene_symbol": "RNPC3"
}